{
  "gene_name": "Integrator complex subunit 1",
  "term_id": "GO:0032039",
  "gene": "UniProtKB:Q8N201",
  "term_label": "integrator complex",
  "gene_symbol": "INTS1"
}